L-lysine transmembrane import into the mitochondrion [GO:0160256] (biological process) Relationships: is_a GO:0170036; is a type of L-lysine transmembrane transport [GO:1903401] Definition: The process in which L-lysine is transported from the cytosol into the mitochondrial matrix. References: PMID:24652292